energy coupled proton transport, down electrochemical gradient [GO:0015985] (biological process) Sources: GOC:mah Definition: The transport of protons across a membrane to generate an electrochemical gradient (proton-motive force) that provides energy for the synthesis of ATP or GTP. Relationships: is_a proton transmembrane transport [GO:1902600] Subtypes: GO:0015987